{
  "gene": "UniProtKB:O75764",
  "gene_name": "Transcription elongation factor A protein 3",
  "gene_symbol": "TCEA3",
  "term_label": "transcription elongation factor activity",
  "term_id": "GO:0003711"
}